{
  "term_label": "DNA-binding transcription factor activity, RNA polymerase II-specific",
  "gene": "UniProtKB:P14653",
  "term_id": "GO:0000981",
  "gene_name": "Homeobox protein Hox-B1",
  "gene_symbol": "HOXB1"
}